protein import into chloroplast thylakoid membrane [GO:0045038] (biological process) Relationships: is a type of protein import [GO:0017038]; is_a GO:0044743; is a type of establishment of protein localization to chloroplast [GO:0072596]; is a type of protein localization to chloroplast [GO:0072598]; is a type of protein localization to membrane [GO:0072657]; is a type of GO:0090150 Also known as: chloroplast thylakoid membrane protein import, protein transport into chloroplast thylakoid membrane Sources: ISBN:0716731363 Definition: The import of proteins into the chloroplast thylakoid membranes. Proteins that are destined for the thylakoid lumen require two uptake-targeting sequences: the first targets the protein to the stroma, and the second targets the protein from the stroma to the thylakoid lumen. Four separate thylakoid-import systems deal with the proteins once they are in the stroma.